cellular response to mycotoxin [GO:0036146] (biological process) Definition: Any process that results in a change in state or activity of a cell (in terms of movement, secretion, enzyme production, gene expression, etc.) as a result of a mycotoxin stimulus. A mycotoxin is a toxic chemical substance produced by fungi. References: PMID:20548963 Sources: GOC:di Relationships: is a type of response to mycotoxin [GO:0010046]; is a type of GO:0097237